{
  "gene_symbol": "SH3GL1",
  "gene": "UniProtKB:Q99961",
  "term_label": "presynapse",
  "gene_name": "Endophilin-A2",
  "term_id": "GO:0098793"
}